curcumin synthase activity [GO:0102106] (molecular function) Definition: Catalysis of the reaction: feruloylacetyl-CoA + feruloyl-CoA(4-) + H2O = curcumin + 2 coenzyme A(4-) + carbon dioxide. Sources: EC:2.3.1.217, GOC:pz Relationships: is a type of acyltransferase activity, transferring groups other than amino-acyl groups [GO:0016747]